deoxynucleoside phosphate kinase activity, ATP as phosphate donor [GO:0047507] (molecular function) Subtypes: dTMP kinase activity [GO:0004798], dCMP kinase activity [GO:0036431], GO:0047506, dGMP kinase activity [GO:0050316], dUMP kinase activity [GO:0120136] Relationships: is a type of phosphotransferase activity, phosphate group as acceptor [GO:0016776]; is a type of nucleobase-containing compound kinase activity [GO:0019205] Definition: Catalysis of the reaction: a 2'-deoxyribonucleoside 5'-phosphate + ATP = a 2'-deoxyribonucleoside 5'-diphosphate + ADP. Also known as: deoxynucleoside-phosphate kinase activity, ATP:deoxynucleoside-phosphate phosphotransferase activity, deoxynucleoside monophosphate kinase activity, deoxynucleoside-5'-monophosphate kinase activity, deoxyribonucleoside monophosphokinase activity Sources: RHEA:11216